{
  "term_id": "GO:0043161",
  "gene_symbol": "PRAMEF5",
  "term_label": "proteasome-mediated ubiquitin-dependent protein catabolic process",
  "gene": "UniProtKB:Q5TYX0",
  "gene_name": "PRAME family member 5"
}